{
  "term_label": "ATP binding",
  "gene": "UniProtKB:P49589",
  "gene_symbol": "CARS1",
  "term_id": "GO:0005524",
  "gene_name": "Cysteine--tRNA ligase, cytoplasmic"
}